{
  "gene_symbol": "KIF5B",
  "gene": "UniProtKB:P33176",
  "gene_name": "Kinesin-1 heavy chain",
  "term_label": "kinesin complex",
  "term_id": "GO:0005871"
}